{
  "gene_symbol": "ADAM10",
  "gene_name": "Disintegrin and metalloproteinase domain-containing protein 10",
  "term_id": "GO:0006509",
  "gene": "UniProtKB:O14672",
  "term_label": "membrane protein ectodomain proteolysis"
}